{
  "gene": "UniProtKB:Q8NI08",
  "term_id": "GO:0006357",
  "gene_symbol": "NCOA7",
  "term_label": "regulation of transcription by RNA polymerase II",
  "gene_name": "Nuclear receptor coactivator 7"
}